vellosimine dehydrogenase activity [GO:0050579] (molecular function) Definition: Catalysis of the reaction: 10-deoxysarpagine + NADP+ = H+ + NADPH + vellosimine. Sources: EC:1.1.1.273, RHEA:20029 Also known as: 10-deoxysarpagine:NADP+ oxidoreductase activity Relationships: is a type of oxidoreductase activity, acting on the CH-OH group of donors, NAD or NADP as acceptor [GO:0016616]